{
  "term_label": "Unknown molecular function",
  "gene_name": "V-set and transmembrane domain-containing protein 2-like protein",
  "gene_symbol": "VSTM2L",
  "term_id": "UNKNOWN:0001",
  "gene": "UniProtKB:Q96N03"
}